kinetoplast [GO:0020023] (cellular component) Definition: A sub-structure within the large single mitochondrion of kinetoplastid parasites and which is closely associated with the flagellar pocket and basal body of the flagellum. Subtypes: antipodal site [GO:0140525] Sources: GOC:mb Relationships: is a type of cellular anatomical structure [GO:0110165]; is part of mitochondrion [GO:0005739]